{
  "gene_symbol": "IGKV1-17",
  "term_label": "immunoglobulin complex",
  "gene_name": "Immunoglobulin kappa variable 1-17",
  "term_id": "GO:0019814",
  "gene": "UniProtKB:P01599"
}